{
  "gene_symbol": "POLDIP3",
  "gene": "UniProtKB:Q9BY77",
  "term_id": "GO:0016973",
  "term_label": "poly(A)+ mRNA export from nucleus",
  "gene_name": "Polymerase delta-interacting protein 3"
}